{
  "gene_symbol": "FAM166C",
  "term_label": "Unknown cellular component",
  "gene_name": "Protein FAM166C",
  "gene": "UniProtKB:A6NJV1",
  "term_id": "UNKNOWN:0003"
}